{
  "gene_symbol": "DHX40",
  "term_label": "mRNA splicing, via spliceosome",
  "gene_name": "Probable ATP-dependent RNA helicase DHX40",
  "gene": "UniProtKB:Q8IX18",
  "term_id": "GO:0000398"
}